{
  "term_id": "GO:0030032",
  "gene_symbol": "ABLIM2",
  "gene_name": "Actin-binding LIM protein 2",
  "term_label": "lamellipodium assembly",
  "gene": "UniProtKB:Q6H8Q1"
}